{
  "term_label": "Unknown cellular component",
  "gene_symbol": "DEPDC4",
  "gene": "UniProtKB:Q8N2C3",
  "gene_name": "DEP domain-containing protein 4",
  "term_id": "UNKNOWN:0003"
}